pronephric distal tubule development [GO:0035777] (biological process) Definition: The process whose specific outcome is the progression of the pronephric distal tubule over time, from its formation to the mature structure. A pronephric nephron tubule is an epithelial tube that is part of the pronephros. References: PMID:18787069 Sources: GOC:mtg_kidney_jan10, GOC:yaf Relationships: is a type of pronephric nephron tubule development [GO:0039020]; is_a distal tubule development [GO:0072017]